{
  "gene_symbol": "LPL",
  "term_id": "GO:0034372",
  "gene": "UniProtKB:P06858",
  "gene_name": "Lipoprotein lipase",
  "term_label": "very-low-density lipoprotein particle remodeling"
}